{
  "gene_name": "GrpE protein homolog 1, mitochondrial",
  "term_label": "adenyl-nucleotide exchange factor activity",
  "gene_symbol": "GRPEL1",
  "term_id": "GO:0000774",
  "gene": "UniProtKB:Q9HAV7"
}